{
  "gene_symbol": "SAG",
  "gene": "UniProtKB:P10523",
  "term_label": "G protein-coupled receptor internalization",
  "gene_name": "S-arrestin",
  "term_id": "GO:0002031"
}